{
  "gene_name": "AP-3 complex subunit sigma-1",
  "term_id": "GO:0016192",
  "gene": "UniProtKB:Q92572",
  "term_label": "vesicle-mediated transport",
  "gene_symbol": "AP3S1"
}